{
  "gene_symbol": "LRRC8E",
  "term_label": "monoatomic ion channel complex",
  "gene_name": "Volume-regulated anion channel subunit LRRC8E",
  "gene": "UniProtKB:Q6NSJ5",
  "term_id": "GO:0034702"
}